gamma-delta T cell activation [GO:0046629] (BP) Definition: The change in morphology and behavior of a gamma-delta T cell resulting from exposure to a mitogen, cytokine, chemokine, cellular ligand, or an antigen for which it is specific. Also known as: gamma-delta T lymphocyte activation, gamma-delta T-cell activation, gamma-delta T-lymphocyte activation Relationships: is a type of T cell activation [GO:0042110] Sources: GOC:add Subtypes: gamma-delta T cell activation involved in immune response [GO:0002290], gamma-delta T cell differentiation [GO:0042492], gamma-delta T cell proliferation [GO:0046630] Regulation: regulated by GO:0046643; negatively regulated by GO:0046644; positively regulated by positive regulation of gamma-delta T cell activation [GO:0046645]